{
  "gene_symbol": "MACIR",
  "term_id": "UNKNOWN:0003",
  "gene_name": "Macrophage immunometabolism regulator",
  "gene": "UniProtKB:Q96GV9",
  "term_label": "Unknown cellular component"
}